{
  "term_label": "embryonic hemopoiesis",
  "term_id": "GO:0035162",
  "gene_name": "Rhombotin-2",
  "gene": "UniProtKB:P25791",
  "gene_symbol": "LMO2"
}